eugenol biosynthetic process [GO:0042855] (biological process) Definition: The chemical reactions and pathways resulting in the formation of eugenol, a colorless, aromatic, liquid hydrocarbon (C10H12O2) found in clove oil. Relationships: is_a phenylpropanoid biosynthetic process [GO:0009699]; is a type of eugenol metabolic process [GO:0042854]; is a type of phenol-containing compound biosynthetic process [GO:0046189]; is_a olefinic compound biosynthetic process [GO:0120255]; is a type of GO:1901503 Sources: GOC:jl Also known as: 4-allyl-2-methoxyphenol biosynthesis, 4-allyl-2-methoxyphenol biosynthetic process, eugenic acid biosynthesis, eugenic acid biosynthetic process, eugenol anabolism, eugenol biosynthesis, eugenol formation, eugenol synthesis